{
  "gene_name": "GLIPR1-like protein 2",
  "term_id": "UNKNOWN:0002",
  "gene_symbol": "GLIPR1L2",
  "term_label": "Unknown biological process",
  "gene": "UniProtKB:Q4G1C9"
}